{
  "gene_symbol": "SH3D19",
  "term_label": "protein-macromolecule adaptor activity",
  "gene": "UniProtKB:Q5HYK7",
  "term_id": "GO:0030674",
  "gene_name": "SH3 domain-containing protein 19"
}